{
  "gene": "UniProtKB:Q8NI51",
  "term_label": "DNA-binding transcription activator activity, RNA polymerase II-specific",
  "gene_symbol": "CTCFL",
  "gene_name": "Transcriptional repressor CTCFL",
  "term_id": "GO:0001228"
}